{
  "term_label": "Unknown cellular component",
  "gene": "UniProtKB:Q8N0Y5",
  "gene_name": "Olfactory receptor 8I2",
  "gene_symbol": "OR8I2",
  "term_id": "UNKNOWN:0003"
}